{
  "gene_symbol": "DAGLA",
  "term_label": "diacylglycerol catabolic process",
  "term_id": "GO:0046340",
  "gene": "UniProtKB:Q9Y4D2",
  "gene_name": "Diacylglycerol lipase-alpha"
}